deoxyuridine catabolic process [GO:0006219] (biological process) Sources: GOC:go_curators Definition: The chemical reactions and pathways resulting in the breakdown of deoxyuridine, 2-deoxyribosyluracil, one of the four major nucleosides of DNA. Relationships: is_a deoxyuridine metabolic process [GO:0046096]; is a type of GO:0046127 Also known as: deoxyuridine breakdown, deoxyuridine catabolism, deoxyuridine degradation